positive regulation of protein localization to lysosome [GO:0150032] (biological process) Sources: GOC:aruk, GOC:bc Definition: Any process that activates or increases the frequency, rate or extent of protein localization to lysosome. Relationships: is a type of GO:0150031; is a type of positive regulation of protein localization [GO:1903829]; positively regulates protein localization to lysosome [GO:0061462]